nematode male tail mating organ morphogenesis [GO:0090597] (biological process) References: PMID:1782863, PMID:18050419, PMID:7409314 Sources: GOC:kmv Relationships: is a type of GO:0048808; is a type of sensory organ morphogenesis [GO:0090596] Definition: The process in which the anatomical structures of the nematode male tail mating organ are generated and organized. The male tail is a sensory organ required for mating and, in C. elegans, consists of ray sensilla, an acellular cuticular fan, a sensory hook, and protracting, copulatory spicules.